{
  "gene_symbol": "GGT7",
  "gene": "UniProtKB:Q9UJ14",
  "gene_name": "Glutathione hydrolase 7",
  "term_id": "GO:0006751",
  "term_label": "glutathione catabolic process"
}